{
  "gene_symbol": "NCKAP5L",
  "term_id": "GO:0007019",
  "term_label": "microtubule depolymerization",
  "gene_name": "Nck-associated protein 5-like",
  "gene": "UniProtKB:Q9HCH0"
}